glutamate synthase complex (NADPH) [GO:0009342] (CC) Definition: A complex that possesses glutamate synthase (NADPH) activity. References: PMID:4565085 Sources: GOC:mah Relationships: is a type of glutamate synthase complex [GO:0031026]